GTPase inhibitor activity [GO:0005095] (molecular function) Also known as: GIP Definition: Stops, prevents or reduces the activity of any enzyme that catalyzes the hydrolysis of GTP to GDP and orthophosphate. Relationships: is a type of GO:0004857; is a type of GTPase regulator activity [GO:0030695]; negatively regulates GTPase activity [GO:0003924] Sources: GOC:ai